{
  "gene_symbol": "RFC5",
  "term_id": "GO:0006281",
  "gene_name": "Replication factor C subunit 5",
  "gene": "UniProtKB:P40937",
  "term_label": "DNA repair"
}